{
  "term_label": "transcription coregulator binding",
  "gene_name": "C-terminal-binding protein 1",
  "term_id": "GO:0001221",
  "gene": "UniProtKB:Q13363",
  "gene_symbol": "CTBP1"
}